alditol catabolic process [GO:0019405] (biological process) Relationships: is a type of carbohydrate catabolic process [GO:0016052]; is a type of GO:0046174 Definition: The chemical reactions and pathways resulting in the breakdown of alditols, any polyhydric alcohol derived from the acyclic form of a monosaccharide by reduction of its aldehyde or keto group to an alcoholic group. Sources: ISBN:0198506732 Also known as: alditol breakdown, alditol catabolism, alditol degradation Subtypes: hexitol catabolic process [GO:0019407], pentitol catabolic process [GO:0019527], glycerol catabolic process [GO:0019563]